{
  "term_id": "GO:0004674",
  "term_label": "protein serine/threonine kinase activity",
  "gene_name": "Nuclear receptor-binding protein 2",
  "gene": "UniProtKB:Q9NSY0",
  "gene_symbol": "NRBP2"
}